{
  "gene_name": "Chromobox protein homolog 7",
  "gene": "UniProtKB:O95931",
  "gene_symbol": "CBX7",
  "term_id": "GO:0000122",
  "term_label": "negative regulation of transcription by RNA polymerase II"
}